regulation of bipolar cell growth [GO:0051516] (biological process) Relationships: is a type of GO:0051510; regulates bipolar cell growth [GO:0042815] Subtypes: negative regulation of bipolar cell growth [GO:0051517], positive regulation of bipolar cell growth [GO:0051518] Definition: Any process that modulates the frequency, rate or extent of bipolar cell growth, polarized growth from both ends of a cell. Sources: GOC:ai